{
  "term_label": "plasma membrane",
  "gene_symbol": "CCNYL1",
  "gene_name": "Cyclin-Y-like protein 1",
  "term_id": "GO:0005886",
  "gene": "UniProtKB:Q8N7R7"
}